{
  "gene_symbol": "TNFRSF1B",
  "gene": "UniProtKB:P20333",
  "gene_name": "Tumor necrosis factor receptor superfamily member 1B",
  "term_label": "tumor necrosis factor binding",
  "term_id": "GO:0043120"
}